{
  "term_label": "Unknown molecular function",
  "gene_name": "Exonuclease mut-7 homolog",
  "gene": "UniProtKB:Q8N9H8",
  "term_id": "UNKNOWN:0001",
  "gene_symbol": "EXD3"
}